{
  "term_id": "GO:0016461",
  "gene_name": "Unconventional myosin-XVIIIb",
  "gene_symbol": "MYO18B",
  "gene": "UniProtKB:Q8IUG5",
  "term_label": "unconventional myosin complex"
}